{
  "term_label": "plasma membrane",
  "gene_name": "Axin-1",
  "gene_symbol": "AXIN1",
  "gene": "UniProtKB:O15169",
  "term_id": "GO:0005886"
}